{
  "gene": "UniProtKB:P63172",
  "term_label": "cytoplasmic dynein complex",
  "term_id": "GO:0005868",
  "gene_symbol": "DYNLT1",
  "gene_name": "Dynein light chain Tctex-type 1"
}